nephron morphogenesis [GO:0072028] (biological process) Definition: The process in which the anatomical structures of the nephron are generated and organized. A nephron is the functional unit of the kidney. Subtypes: pronephric nephron morphogenesis [GO:0039007], GO:0061228, GO:0072273 Relationships: is a type of anatomical structure morphogenesis [GO:0009653]; is part of kidney morphogenesis [GO:0060993]; is part of GO:0072006 Sources: GOC:mtg_kidney_jan10